{
  "gene_symbol": "MGRN1",
  "term_label": "endosome to lysosome transport",
  "term_id": "GO:0008333",
  "gene_name": "E3 ubiquitin-protein ligase MGRN1",
  "gene": "UniProtKB:O60291"
}